intratendonous ossification [GO:0036077] (biological process) Note: Tendonous ossification may occur via replacement ossification or metaplastic ossification or both in any one instance. Sources: GO_REF:0000034 Definition: Ossification wherein bone tissue forms within tendonous tissue. Relationships: is a type of GO:0001503